{
  "term_id": "GO:0005634",
  "gene_name": "NKAP-like protein",
  "term_label": "nucleus",
  "gene": "UniProtKB:Q5M9Q1",
  "gene_symbol": "NKAPL"
}